large intestinal transit [GO:0120056] (BP) Definition: Migration of ingested material along the length of the large intestine. Also known as: colon transit, colonic transit, large bowel transit, large intestine transit Relationships: is a type of intestinal motility [GO:0120054] References: PMID:28157109 Sources: GOC:sl